protein maturation [GO:0051604] (biological process) Relationships: is a type of GO:0019538; is part of gene expression [GO:0010467] Subtypes: N-terminal protein amino acid acetylation [GO:0006474], peptide pheromone maturation [GO:0007323], GO:0008612, protein lipoylation [GO:0009249], attachment of GPI anchor to protein [GO:0016255], GO:0016485, protein-tetrapyrrole linkage [GO:0017006], protein activation cascade [GO:0072376], CAAX-box protein maturation [GO:0080120], GPI anchored protein biosynthesis [GO:0180046] Regulation: RO_0002211 by regulation of protein maturation [GO:1903317]; RO_0002212 by GO:1903318; positively regulated by positive regulation of protein maturation [GO:1903319] Definition: Any process leading to the attainment of the full functional capacity of a protein. Sources: GOC:ai